{
  "term_label": "cortical endoplasmic reticulum",
  "term_id": "GO:0032541",
  "gene_name": "Protein ARV1",
  "gene_symbol": "ARV1",
  "gene": "UniProtKB:Q9H2C2"
}